{
  "term_label": "gap junction-mediated intercellular transport",
  "term_id": "GO:1990349",
  "gene_symbol": "GJB6",
  "gene": "UniProtKB:O95452",
  "gene_name": "Gap junction beta-6 protein"
}